negative regulation of antigen receptor-mediated signaling pathway [GO:0050858] (biological process) Subtypes: negative regulation of B cell receptor signaling pathway [GO:0050859], negative regulation of T cell receptor signaling pathway [GO:0050860] Relationships: is a type of negative regulation of immune system process [GO:0002683]; is a type of negative regulation of signal transduction [GO:0009968]; is_a regulation of antigen receptor-mediated signaling pathway [GO:0050854]; negatively regulates antigen receptor-mediated signaling pathway [GO:0050851] Also known as: down regulation of antigen receptor-mediated signaling pathway, down-regulation of antigen receptor-mediated signaling pathway, downregulation of antigen receptor-mediated signaling pathway, negative regulation of antigen receptor mediated signalling pathway, inhibition of antigen receptor-mediated signaling pathway Definition: Any process that stops, prevents, or reduces the frequency, rate or extent of signaling pathways initiated by the cross-linking of an antigen receptor on a B- or T cell. Sources: GOC:ai